aspartate racemase activity [GO:0047689] (molecular function) Definition: Catalysis of the reaction: L-aspartate = D-aspartate. Sources: EC:5.1.1.13, RHEA:14973 Also known as: D-aspartate racemase activity Relationships: is a type of GO:0047661